{
  "gene_name": "Phosphatidylinositol-glycan biosynthesis class W protein",
  "gene_symbol": "PIGW",
  "gene": "UniProtKB:Q7Z7B1",
  "term_id": "GO:0006506",
  "term_label": "GPI anchor biosynthetic process"
}